{
  "gene_name": "Zinc finger MYND domain-containing protein 11",
  "gene_symbol": "ZMYND11",
  "term_id": "GO:0009966",
  "term_label": "regulation of signal transduction",
  "gene": "UniProtKB:Q15326"
}